{
  "gene_name": "UDP-glucuronosyltransferase 1-6",
  "gene": "UniProtKB:P19224",
  "term_label": "enzyme binding",
  "term_id": "GO:0019899",
  "gene_symbol": "UGT1A6"
}